pentosyltransferase activity [GO:0016763] (molecular function) Sources: GOC:jl Subtypes: imidazoleglycerol-phosphate synthase activity [GO:0000107], GO:0003879, NAD+ poly-ADP-ribosyltransferase activity [GO:0003950], amidophosphoribosyltransferase activity [GO:0004044], anthranilate phosphoribosyltransferase activity [GO:0004048], nicotinate-nucleotide diphosphorylase (carboxylating) activity [GO:0004514], GO:0004588, purine-nucleoside phosphorylase activity [GO:0004731], uracil phosphoribosyltransferase activity [GO:0004845], tRNA-guanosine(34) queuine transglycosylase activity [GO:0008479], GO:0008939, pyrimidine-nucleoside phosphorylase activity [GO:0016154], NAD+-dinitrogen-reductase ADP-D-ribosyltransferase activity [GO:0030701], xylosyltransferase activity [GO:0042285], tRNA adenosine(64)-2'-O-ribosylphosphate transferase activity [GO:0043399], beta-ribofuranosylaminobenzene 5'-phosphate synthase activity [GO:0043793], 7-cyano-7-deazaguanine tRNA-ribosyltransferase activity [GO:0043867], GO:0044102, nicotinamide phosphoribosyltransferase activity [GO:0047280], dioxotetrahydropyrimidine phosphoribosyltransferase activity [GO:0047281], GO:0047282, NAD+-diphthamide ADP-ribosyltransferase activity [GO:0047286], GO:0047517, flavone apiosyltransferase activity [GO:0047892], guanosine phosphorylase activity [GO:0047975], nucleoside deoxyribosyltransferase activity [GO:0050144], nucleoside ribosyltransferase activity [GO:0050147], urate-ribonucleotide phosphorylase activity [GO:0050384], arabinosyltransferase activity [GO:0052636], GO:0099621, GO:0102580, GO:0102983, 4-amino-4-deoxy-L-arabinose transferase activity [GO:0103015], purine phosphoribosyltransferase activity [GO:0106130], NAD DNA ADP-ribosyltransferase activity [GO:0140294], GO:0160205, NAD+-protein mono-ADP-ribosyltransferase activity [GO:1990404], GO:1990585 Also known as: transferase activity, transferring pentosyl groups Definition: Catalysis of the transfer of a pentosyl group from one compound (donor) to another (acceptor). Relationships: is_a GO:0016757